{
  "term_label": "cytoplasm",
  "term_id": "GO:0005737",
  "gene_symbol": "CIROP",
  "gene": "UniProtKB:A0A1B0GTW7",
  "gene_name": "Ciliated left-right organizer metallopeptidase"
}